CD8-positive, alpha-beta T cell proliferation [GO:0035740] (biological process) Relationships: is a type of GO:0036037; is a type of alpha-beta T cell proliferation [GO:0046633] Sources: CL:0000625, GOC:BHF Subtypes: GO:0035742 Definition: The expansion of a CD8-positive, alpha-beta T cell population by cell division. Regulation: regulated by regulation of CD8-positive, alpha-beta T cell proliferation [GO:2000564]; negatively regulated by negative regulation of CD8-positive, alpha-beta T cell proliferation [GO:2000565]; positively regulated by positive regulation of CD8-positive, alpha-beta T cell proliferation [GO:2000566]